{
  "term_label": "nucleus",
  "gene_name": "AKT-interacting protein",
  "gene": "UniProtKB:Q9H8T0",
  "term_id": "GO:0005634",
  "gene_symbol": "AKTIP"
}